histone methyltransferase complex [GO:0035097] (cellular component) Relationships: is a type of methyltransferase complex [GO:0034708]; is a type of nuclear protein-containing complex [GO:0140513]; is part of nucleoplasm [GO:0005654] Subtypes: ESC/E(Z) complex [GO:0035098], CLRC complex [GO:0043494], MLL1/2 complex [GO:0044665], MLL3/4 complex [GO:0044666], Set1C/COMPASS complex [GO:0048188], GO:0070311 Sources: GOC:bf Definition: A multimeric complex that is able to catalyze the addition of methyl groups to histone proteins.